{
  "gene": "UniProtKB:Q9Y6M0",
  "gene_name": "Testisin",
  "term_id": "GO:0004252",
  "gene_symbol": "PRSS21",
  "term_label": "serine-type endopeptidase activity"
}